{
  "gene_symbol": "SLC4A5",
  "term_label": "bicarbonate transport",
  "gene_name": "Electrogenic sodium bicarbonate cotransporter 4",
  "term_id": "GO:0015701",
  "gene": "UniProtKB:Q9BY07"
}